{
  "gene_symbol": "PIK3R2",
  "gene": "UniProtKB:O00459",
  "term_label": "phosphatidylinositol 3-kinase complex, class IA",
  "gene_name": "Phosphatidylinositol 3-kinase regulatory subunit beta",
  "term_id": "GO:0005943"
}